{
  "gene_symbol": "KICS2",
  "term_id": "GO:0061462",
  "gene_name": "KICSTOR subunit 2",
  "term_label": "protein localization to lysosome",
  "gene": "UniProtKB:Q96MD2"
}